{
  "gene": "UniProtKB:Q6ZS86",
  "term_id": "GO:0046167",
  "gene_symbol": "GK5",
  "term_label": "glycerol-3-phosphate biosynthetic process",
  "gene_name": "Putative glycerol kinase 5"
}